{
  "term_id": "GO:0045739",
  "term_label": "positive regulation of DNA repair",
  "gene_symbol": "UIMC1",
  "gene": "UniProtKB:Q96RL1",
  "gene_name": "BRCA1-A complex subunit RAP80"
}